{
  "term_label": "ubiquitin protein ligase activity",
  "gene": "UniProtKB:Q9H2S5",
  "gene_symbol": "RNF39",
  "gene_name": "RING finger protein 39",
  "term_id": "GO:0061630"
}